{
  "gene_symbol": "FAM157A",
  "gene_name": "Putative protein FAM157A",
  "gene": "UniProtKB:C9JC47",
  "term_id": "UNKNOWN:0003",
  "term_label": "Unknown cellular component"
}